{
  "gene_name": "Activin receptor type-1",
  "term_label": "cell differentiation",
  "gene_symbol": "ACVR1",
  "term_id": "GO:0030154",
  "gene": "UniProtKB:Q04771"
}